{
  "gene_name": "Oxygen-regulated protein 1",
  "term_label": "photoreceptor connecting cilium",
  "gene_symbol": "RP1",
  "term_id": "GO:0032391",
  "gene": "UniProtKB:P56715"
}